{
  "gene_name": "Fibronectin type III domain-containing protein 1",
  "gene": "UniProtKB:Q4ZHG4",
  "term_id": "UNKNOWN:0002",
  "term_label": "Unknown biological process",
  "gene_symbol": "FNDC1"
}